{
  "gene_symbol": "GABRA2",
  "term_label": "postsynapse",
  "gene_name": "Gamma-aminobutyric acid receptor subunit alpha-2",
  "term_id": "GO:0098794",
  "gene": "UniProtKB:P47869"
}